{
  "gene": "UniProtKB:P35236",
  "term_label": "signal transduction",
  "gene_symbol": "PTPN7",
  "term_id": "GO:0007165",
  "gene_name": "Tyrosine-protein phosphatase non-receptor type 7"
}